regulation of mitochondrial mRNA stability [GO:0044528] (biological process) Definition: Any process that modulates the propensity of mitochondrial mRNA molecules to degradation. Includes processes that both stabilize and destabilize mitochondrial mRNAs. Sources: GOC:al, GOC:jl Relationships: is a type of GO:0043488